{
  "gene_name": "Putative STAG3-like protein 4",
  "gene_symbol": "STAG3L4",
  "term_label": "Unknown molecular function",
  "term_id": "UNKNOWN:0001",
  "gene": "UniProtKB:Q8TBR4"
}